{
  "term_label": "RNA polymerase II transcription regulator complex",
  "gene": "UniProtKB:P37231",
  "term_id": "GO:0090575",
  "gene_symbol": "PPARG",
  "gene_name": "Peroxisome proliferator-activated receptor gamma"
}